negative regulation of cell adhesion molecule production [GO:0060354] (BP) Definition: Any process that decreases the rate, frequency or extent of cell adhesion molecule production. Cell adhesion molecule production is the appearance of a cell adhesion molecule as a result of its biosynthesis or a decrease in its catabolism. Sources: GOC:BHF, GOC:rl Relationships: is a type of negative regulation of cellular process [GO:0048523]; is a type of regulation of cell adhesion molecule production [GO:0060353]; negatively regulates cell adhesion molecule production [GO:0060352]